{
  "gene_symbol": "ACTR3",
  "term_id": "GO:0034314",
  "term_label": "Arp2/3 complex-mediated actin nucleation",
  "gene": "UniProtKB:P61158",
  "gene_name": "Actin-related protein 3"
}